{
  "term_label": "Unknown molecular function",
  "gene_name": "Putative uncharacterized protein encoded by LINC00526",
  "gene_symbol": "LINC00526",
  "term_id": "UNKNOWN:0001",
  "gene": "UniProtKB:Q96FQ7"
}